{
  "term_label": "positive regulation of membrane tubulation",
  "gene_name": "Arf-GAP with SH3 domain, ANK repeat and PH domain-containing protein 1",
  "gene_symbol": "ASAP1",
  "term_id": "GO:1903527",
  "gene": "UniProtKB:Q9ULH1"
}